{
  "term_label": "Unknown cellular component",
  "gene_name": "Cancer-related nucleoside-triphosphatase",
  "gene_symbol": "NTPCR",
  "gene": "UniProtKB:Q9BSD7",
  "term_id": "UNKNOWN:0003"
}